{
  "gene_name": "Nuclear factor related to kappa-B-binding protein",
  "term_label": "Unknown biological process",
  "gene_symbol": "NFRKB",
  "term_id": "UNKNOWN:0002",
  "gene": "UniProtKB:Q6P4R8"
}